{
  "gene": "UniProtKB:P05388",
  "gene_symbol": "RPLP0",
  "term_id": "GO:0070180",
  "term_label": "large ribosomal subunit rRNA binding",
  "gene_name": "Large ribosomal subunit protein uL10"
}